regulation of long-chain fatty acid import across plasma membrane [GO:0010746] (biological process) Definition: Any process that modulates the rate, frequency or extent of plasma membrane long-chain fatty acid transport. Plasma membrane long-chain fatty acid transport is the directed movement of long-chain fatty acids across the plasma membrane. A long-chain fatty acid has an aliphatic tail containing 13 to 22 carbons. Sources: GOC:BHF, GOC:dph, GOC:tb Also known as: regulation of plasma membrane long-chain fatty acid transport Note: While there is not universal consensus on the lengths of short-, medium-, long- and very-long-chain fatty acids, the GO uses the definitions in ChEBI (see CHEBI:26666, CHEBI:59554, CHEBI:15904 and CHEBI:27283). Relationships: is a type of GO:0034762; is a type of regulation of long-chain fatty acid import into cell [GO:0140212]; regulates GO:0015911 Subtypes: GO:0010747, negative regulation of long-chain fatty acid import across plasma membrane [GO:0010748]